{
  "term_id": "GO:0005886",
  "gene": "UniProtKB:Q9UQV4",
  "gene_symbol": "LAMP3",
  "term_label": "plasma membrane",
  "gene_name": "Lysosome-associated membrane glycoprotein 3"
}